{
  "gene": "UniProtKB:Q8N4L4",
  "term_label": "cytoplasm",
  "gene_name": "Spermatid maturation protein 1",
  "term_id": "GO:0005737",
  "gene_symbol": "SPEM1"
}